{
  "term_label": "proteolysis",
  "gene": "UniProtKB:Q8TE56",
  "gene_symbol": "ADAMTS17",
  "term_id": "GO:0006508",
  "gene_name": "A disintegrin and metalloproteinase with thrombospondin motifs 17"
}